{
  "gene_name": "Gamma-tubulin complex component 3",
  "gene_symbol": "TUBGCP3",
  "term_id": "GO:0000930",
  "gene": "UniProtKB:Q96CW5",
  "term_label": "gamma-tubulin complex"
}